{
  "gene_symbol": "CREB3L2",
  "term_id": "UNKNOWN:0003",
  "gene_name": "Cyclic AMP-responsive element-binding protein 3-like protein 2",
  "gene": "UniProtKB:Q70SY1",
  "term_label": "Unknown cellular component"
}